{
  "gene": "UniProtKB:P59827",
  "term_label": "Unknown molecular function",
  "term_id": "UNKNOWN:0001",
  "gene_name": "BPI fold-containing family B member 4",
  "gene_symbol": "BPIFB4"
}